{
  "term_id": "GO:0005886",
  "gene": "UniProtKB:P49407",
  "term_label": "plasma membrane",
  "gene_name": "Beta-arrestin-1",
  "gene_symbol": "ARRB1"
}